strigolactone metabolic process [GO:1901600] (biological process) Definition: The chemical reactions and pathways involving strigolactone. Sources: GOC:TermGenie Also known as: strigolactone metabolism Relationships: is a type of sesquiterpenoid metabolic process [GO:0006714]; is a type of lactone metabolic process [GO:1901334] Subtypes: strigolactone biosynthetic process [GO:1901601]